{
  "gene_name": "Putative WAS protein family homolog 3",
  "term_id": "GO:0071203",
  "gene_symbol": "WASH3P",
  "gene": "UniProtKB:C4AMC7",
  "term_label": "WASH complex"
}